cis-abienol biosynthetic process [GO:1902246] (biological process) Also known as: cis-abienol anabolism, cis-abienol biosynthesis, cis-abienol formation, cis-abienol synthesis References: PMID:22672125 Sources: GOC:TermGenie Relationships: is_a diterpenoid biosynthetic process [GO:0016102]; is a type of GO:1902645 Definition: The chemical reactions and pathways resulting in the formation of cis-abienol.